{
  "term_id": "UNKNOWN:0001",
  "term_label": "Unknown molecular function",
  "gene_name": "Double C2-like domain-containing protein beta",
  "gene": "UniProtKB:Q14184",
  "gene_symbol": "DOC2B"
}